{
  "gene": "UniProtKB:Q15050",
  "term_label": "Unknown molecular function",
  "gene_name": "Ribosome biogenesis regulatory protein homolog",
  "term_id": "UNKNOWN:0001",
  "gene_symbol": "RRS1"
}